proteinase-activated receptor activity [GO:0001648] (molecular function) Relationships: is a type of GO:0008528 References: PMID:11356985, PMID:33742547 Sources: GOC:mah Subtypes: thrombin-activated receptor activity [GO:0015057] Also known as: protease-activated receptor activity, proteinase activated receptor activity Definition: A G protein-coupled receptor activity that is activated by cleavage by a serine protease, exposing a tethered ligand corresponding to the new N-terminus, which binds to the receptor and activates it.